acetone carboxylase activity [GO:0018710] (molecular function) Relationships: is a type of GO:0016885 Also known as: acetone:carbon-dioxide ligase (AMP-forming) Sources: EC:6.4.1.6, RHEA:18385 Definition: Catalysis of the reaction: acetone + ATP + CO2 + 2 H2O = acetoacetate + AMP + 4 H+ + 2 phosphate.